negative regulation of glucocorticoid secretion [GO:2000850] (biological process) Relationships: is a type of negative regulation of corticosteroid hormone secretion [GO:2000847]; is a type of GO:2000849; negatively regulates glucocorticoid secretion [GO:0035933] Sources: GOC:sl Definition: Any process that stops, prevents or reduces the frequency, rate or extent of glucocorticoid secretion. Subtypes: negative regulation of cortisol secretion [GO:0051463], GO:2000853